cell tip [GO:0051286] (cellular component) Note: Note that this term differs from 'cell pole ; GO:0060187' in that it is applicable to the thin ends of elongated cells, such as the ends of axons or dendrites. Also known as: cell end Relationships: is_a cell pole [GO:0060187] Sources: GOC:ai, GOC:mah Definition: The region at the end of the longest axis of a cylindrical or elongated cell. Subtypes: hyphal tip [GO:0001411], root hair tip [GO:0035619], growing cell tip [GO:0035838], non-growing cell tip [GO:0035839], mating projection tip [GO:0043332]